tooth replacement [GO:0061648] (biological process) References: PMID:15170864 Sources: GOC:dph Definition: The process whose specific outcome is the replacement of an existing tooth with another tooth. Relationships: is_a odontogenesis [GO:0042476]